{
  "gene_name": "Protein farnesyltransferase_geranylgeranyltransferase type-1 subunit alpha",
  "term_id": "GO:0005965",
  "gene": "UniProtKB:P49354",
  "gene_symbol": "FNTA",
  "term_label": "protein farnesyltransferase complex"
}